anandamide 8,9 epoxidase activity [GO:0062187] (molecular function) References: PMID:21289075 Sources: RHEA:53140 Relationships: is a type of anandamide epoxidase activity [GO:0062186] Definition: Catalysis of the reaction: N-(5Z,8Z,11Z,14Z-eicosatetraenoyl)-ethanolamine + O2 + reduced [NADPH--hemoprotein reductase] = H+ + H2O + N-(8,9-epoxy-5Z,11Z,14Z-eicosatrienoyl)-ethanolamine + oxidized [NADPH--hemoprotein reductase].